RNA polymerase II CTD heptapeptide repeat S5 kinase activity [GO:0140836] (molecular function) Definition: Catalysis of the reaction: ATP + RNA polymerase II large subunit CTD heptapeptide repeat (consensus YSPTSPS) = ADP + H+ + RNA polymerase II large subunit phosphoserine (position 5). References: PMID:28248323 Also known as: RNA polymerase II C-terminal domain S5 kinase activity Relationships: is a type of RNA polymerase II CTD heptapeptide repeat kinase activity [GO:0008353]